{
  "term_id": "GO:0004825",
  "gene_symbol": "MARS2",
  "gene": "UniProtKB:Q96GW9",
  "term_label": "methionine-tRNA ligase activity",
  "gene_name": "Methionine--tRNA ligase, mitochondrial"
}